negative regulation of snRNA pseudouridine synthesis [GO:1905357] (biological process) Also known as: down regulation of snRNA pseudouridine synthesis, down-regulation of snRNA pseudouridine synthesis, downregulation of snRNA pseudouridine synthesis, inhibition of snRNA pseudouridine synthesis References: PMID:27268497 Sources: GOC:TermGenie, GO_REF:0000058 Relationships: is a type of negative regulation of RNA metabolic process [GO:0051253]; is a type of GO:1905356; negatively regulates GO:0031120 Definition: Any process that stops, prevents or reduces the frequency, rate or extent of snRNA pseudouridine synthesis.